{
  "gene_name": "Large ribosomal subunit protein uL1",
  "term_id": "GO:0022625",
  "gene": "UniProtKB:P62906",
  "gene_symbol": "RPL10A",
  "term_label": "cytosolic large ribosomal subunit"
}